{
  "gene_symbol": "CASP12",
  "term_id": "UNKNOWN:0001",
  "gene_name": "Inactive caspase-12",
  "gene": "UniProtKB:Q6UXS9",
  "term_label": "Unknown molecular function"
}